{
  "gene_symbol": "FBXO22",
  "term_id": "GO:0048742",
  "gene_name": "F-box only protein 22",
  "term_label": "regulation of skeletal muscle fiber development",
  "gene": "UniProtKB:Q8NEZ5"
}